granulocyte activation [GO:0036230] (biological process) Sources: CL:0000094, GOC:nhn Subtypes: neutrophil activation [GO:0042119], eosinophil activation [GO:0043307], GO:0045575 Definition: The change in morphology and behavior of a granulocyte resulting from exposure to a cytokine, chemokine, cellular ligand, or soluble factor. Relationships: is a type of myeloid leukocyte activation [GO:0002274]